{
  "gene": "UniProtKB:Q96DL1",
  "gene_name": "NXPE family member 2",
  "gene_symbol": "NXPE2",
  "term_label": "Unknown cellular component",
  "term_id": "UNKNOWN:0003"
}